symbiont-mediated perturbation of host vesicle-mediated transport [GO:1990215] (biological process) Relationships: is a type of symbiont-mediated perturbation of host cellular process [GO:0044068] Definition: A process in which a symbiont alters or subverts vesicle-mediated transport in the host organism. The host is defined as the larger of the organisms involved in a symbiotic interaction. Also known as: negative regulation by symbiont of host intracellular transport, symbiont-mediated perturbation of host endosomal trafficking References: PMID:22319451, PMID:24248335, PMID:30893609, PMID:31492901 Subtypes: GO:0044077, symbiont-mediated suppression of host exocytosis [GO:0141157]